protein-glycine ligase activity [GO:0070735] (molecular function) Relationships: is a type of GO:0016881; is a type of GO:0140096 Subtypes: protein-glycine ligase activity, initiating [GO:0070736], GO:0070737, tubulin-glycine ligase activity [GO:0070738] Definition: Catalysis of the reaction: ATP + glycine + L-glutamyl-[protein] = ADP + glycyl-L-glutamyl-[protein] + H+ + phosphate. Also known as: protein glycylase activity Sources: RHEA:67180